{
  "gene_symbol": "RAC1",
  "term_label": "cytoplasmic vesicle",
  "gene_name": "Ras-related C3 botulinum toxin substrate 1",
  "gene": "UniProtKB:P63000",
  "term_id": "GO:0031410"
}